low-affinity IgA receptor activity [GO:0002171] (molecular function) Also known as: low affinity IgA receptor activity Relationships: is a type of IgA receptor activity [GO:0019766] Definition: Combining with low affinity with an immunoglobulin of an IgA isotype via the Fc region, and transmitting the signal from one side of the membrane to the other to initiate a change in cell activity. Sources: GOC:hjd, GOC:signaling